spontaneous neurotransmitter secretion [GO:0061669] (biological process) Relationships: is a type of neurotransmitter secretion [GO:0007269]; is part of spontaneous synaptic transmission [GO:0098814] Regulation: regulated by regulation of spontaneous neurotransmitter secretion [GO:1904048]; negatively regulated by negative regulation of spontaneous neurotransmitter secretion [GO:1904049]; positively regulated by positive regulation of spontaneous neurotransmitter secretion [GO:1904050] References: PMID:21334193 Sources: GOC:PARL, GOC:dph, GOC:pad Also known as: stimulus-independent neurotransmitter secretion Definition: Neurotransmitter secretion that occurs in the absence of the action of a secretagogue or a presynaptic action potential.